{
  "gene_name": "Ribulose-phosphate 3-epimerase",
  "gene_symbol": "RPE",
  "term_id": "GO:0005975",
  "gene": "UniProtKB:Q96AT9",
  "term_label": "carbohydrate metabolic process"
}